{
  "gene_symbol": "ERP44",
  "gene_name": "Endoplasmic reticulum resident protein 44",
  "term_label": "protein folding",
  "gene": "UniProtKB:Q9BS26",
  "term_id": "GO:0006457"
}